transport across blood-cerebrospinal fluid barrier [GO:0150195] (biological process) Definition: The directed movement of substances (e.g. macromolecules, small molecules, ions) through the blood-cerebrospinal fluid barrier. References: PMID:21349151 Sources: GOC:aruk, GOC:bc Relationships: is a type of vascular transport [GO:0010232] Also known as: transport across BCSFB, transport across blood-CSF barrier, transport across blood/CSF barrier, transport across blood/cerebrospinal fluid barrier Subtypes: copper ion transport across blood-cerebrospinal fluid barrier [GO:0097717]